{
  "term_label": "nucleus",
  "term_id": "GO:0005634",
  "gene": "UniProtKB:P0C7X2",
  "gene_name": "Zinc finger protein 688",
  "gene_symbol": "ZNF688"
}